{
  "gene_name": "Lipid transferase CIDEB",
  "term_label": "lipid droplet fusion",
  "gene": "UniProtKB:Q9UHD4",
  "term_id": "GO:0160077",
  "gene_symbol": "CIDEB"
}